{
  "term_label": "focal adhesion",
  "gene": "UniProtKB:Q9HBI1",
  "gene_name": "Beta-parvin",
  "term_id": "GO:0005925",
  "gene_symbol": "PARVB"
}